arachidonate monooxygenase activity [GO:0008391] (molecular function) Also known as: arachidonic acid monooxygenase activity, cytochrome P450 CYP2B19 Subtypes: arachidonate epoxygenase activity [GO:0008392] Sources: GOC:mah Definition: Catalysis of the incorporation of one atom from molecular oxygen into arachidonic acid and the reduction of the other atom of oxygen to water. Relationships: is a type of monooxygenase activity [GO:0004497]; is a type of oxidoreductase activity, acting on paired donors, with incorporation or reduction of molecular oxygen [GO:0016705]